{
  "term_label": "TSC1-TSC2 complex binding",
  "term_id": "GO:0062078",
  "gene_name": "TBC1 domain family member 7",
  "gene_symbol": "TBC1D7",
  "gene": "UniProtKB:Q9P0N9"
}